{
  "gene_symbol": "ZNF16",
  "term_label": "RNA polymerase II cis-regulatory region sequence-specific DNA binding",
  "gene_name": "Zinc finger protein 16",
  "term_id": "GO:0000978",
  "gene": "UniProtKB:P17020"
}